cardiac neuron fate commitment [GO:0060960] (biological process) Sources: GOC:mtg_heart Definition: The process in which the developmental fate of a cell becomes restricted such that it will develop into a neuron of the heart. Relationships: is a type of neuron fate commitment [GO:0048663]; is a type of cardiac cell fate commitment [GO:0060911]; is part of cardiac neuron differentiation [GO:0060945] Also known as: heart neuron fate commitment